prothylakoid membrane [GO:0042650] (cellular component) Definition: The membrane of prothylakoids, underdeveloped thylakoids found in etioplasts, lacking competent photosynthetic membranes. References: PMID:11532175 Sources: GOC:jl Relationships: is a type of plastid thylakoid membrane [GO:0055035]; BFO_0000050 prothylakoid [GO:0042649]